{
  "gene_symbol": "GFUS",
  "term_id": "UNKNOWN:0002",
  "gene": "UniProtKB:Q13630",
  "term_label": "Unknown biological process",
  "gene_name": "GDP-L-fucose synthase"
}